{
  "gene_symbol": "TRAJ45",
  "gene": "UniProtKB:A0A075B6X0",
  "term_label": "Unknown cellular component",
  "term_id": "UNKNOWN:0003",
  "gene_name": "T cell receptor alpha joining 45 (Fragment)"
}